{
  "gene": "UniProtKB:P55058",
  "term_label": "extracellular space",
  "gene_symbol": "PLTP",
  "term_id": "GO:0005615",
  "gene_name": "Phospholipid transfer protein"
}